{
  "gene": "UniProtKB:Q96BP2",
  "term_id": "UNKNOWN:0002",
  "term_label": "Unknown biological process",
  "gene_symbol": "CHCHD1",
  "gene_name": "Small ribosomal subunit protein mS37"
}